protein-phycocyanobilin linkage [GO:0017009] (biological process) Sources: RESID:AA0131 Definition: The linkage of the chromophore phycocyanobilin to phycocyanin or allophycocyanin. Relationships: is a type of protein-bilin linkage [GO:0017007]